{
  "gene_symbol": "ATG4C",
  "term_id": "GO:0000045",
  "gene_name": "Cysteine protease ATG4C",
  "term_label": "autophagosome assembly",
  "gene": "UniProtKB:Q96DT6"
}